{
  "term_id": "GO:0003887",
  "gene": "UniProtKB:Q9UBT6",
  "gene_name": "DNA polymerase kappa",
  "gene_symbol": "POLK",
  "term_label": "DNA-directed DNA polymerase activity"
}